{
  "term_label": "cysteine-type endopeptidase inhibitor activity involved in apoptotic process",
  "term_id": "GO:0043027",
  "gene_symbol": "TNFAIP8",
  "gene_name": "Tumor necrosis factor alpha-induced protein 8",
  "gene": "UniProtKB:O95379"
}